{
  "gene": "UniProtKB:Q5GH73",
  "gene_symbol": "XKR6",
  "term_label": "apoptotic process involved in development",
  "gene_name": "XK-related protein 6",
  "term_id": "GO:1902742"
}